{
  "gene": "UniProtKB:Q9BXX2",
  "gene_name": "Ankyrin repeat domain-containing protein 30B",
  "gene_symbol": "ANKRD30B",
  "term_id": "UNKNOWN:0002",
  "term_label": "Unknown biological process"
}